{
  "gene": "UniProtKB:Q96PF2",
  "gene_symbol": "TSSK2",
  "term_id": "UNKNOWN:0003",
  "gene_name": "Testis-specific serine_threonine-protein kinase 2",
  "term_label": "Unknown cellular component"
}